{
  "gene_name": "Histone H2B type 2-F",
  "gene": "UniProtKB:Q5QNW6",
  "term_label": "extracellular space",
  "gene_symbol": "H2BC18",
  "term_id": "GO:0005615"
}